negative regulation of transmission of nerve impulse [GO:0051970] (biological process) Subtypes: negative regulation of neuronal action potential [GO:1904456] Sources: GOC:ai Definition: Any process that stops, prevents, or reduces the frequency, rate or extent of transmission of a nerve impulse, the sequential electrochemical polarization and depolarization that travels across the membrane of a neuron in response to stimulation. Also known as: down regulation of transmission of nerve impulse, down-regulation of transmission of nerve impulse, downregulation of transmission of nerve impulse, negative regulation of conduction of nerve impulse, inhibition of transmission of nerve impulse Relationships: is a type of negative regulation of cell communication [GO:0010648]; is a type of negative regulation of nervous system process [GO:0031645]; is a type of regulation of transmission of nerve impulse [GO:0051969]; negatively regulates transmission of nerve impulse [GO:0019226]